{
  "term_label": "Swr1 complex",
  "gene_name": "RuvB-like 2",
  "term_id": "GO:0000812",
  "gene_symbol": "RUVBL2",
  "gene": "UniProtKB:Q9Y230"
}